{
  "term_id": "GO:0045202",
  "term_label": "synapse",
  "gene_symbol": "ADORA3",
  "gene": "UniProtKB:P0DMS8",
  "gene_name": "Adenosine receptor A3"
}